regulation of calcium ion transport [GO:0051924] (biological process) Relationships: is a type of regulation of metal ion transport [GO:0010959]; regulates calcium ion transport [GO:0006816] Definition: Any process that modulates the frequency, rate or extent of the directed movement of calcium ions into, out of or within a cell, or between cells, by means of some agent such as a transporter or pore. Sources: GOC:ai Subtypes: negative regulation of calcium ion transport [GO:0051926], positive regulation of calcium ion transport [GO:0051928], GO:0090279, regulation of calcium ion import into sarcoplasmic reticulum [GO:1902080], GO:1903169, regulation of store-operated calcium entry [GO:2001256] Also known as: regulation of calcium transport